FMN adenylyltransferase activity [GO:0003919] (molecular function) Also known as: ATP:FMN adenylyltransferase activity, FAD diphosphorylase activity, FAD pyrophosphorylase activity, FAD synthetase activity, adenosine triphosphate-riboflavin mononucleotide transadenylase activity, adenosine triphosphate-riboflavine mononucleotide transadenylase activity, flavin adenine dinucleotide synthetase activity, riboflavin adenine dinucleotide pyrophosphorylase activity, riboflavin mononucleotide adenylyltransferase activity, riboflavine adenine dinucleotide adenylyltransferase activity Relationships: is a type of adenylyltransferase activity [GO:0070566] Definition: Catalysis of the reaction: ATP + FMN = diphosphate + FAD. Sources: EC:2.7.7.2, RHEA:17237